{
  "gene_symbol": "LIN7C",
  "gene_name": "Protein lin-7 homolog C",
  "term_label": "MPP7-DLG1-LIN7 complex",
  "gene": "UniProtKB:Q9NUP9",
  "term_id": "GO:0097025"
}